protein-phycoerythrobilin linkage [GO:0017011] (biological process) Definition: The linkage of the chromophore phycoerythrobilin to phycoerythrins. Relationships: is a type of GO:0017007 Sources: RESID:AA0132, RESID:AA0259